ATPase inhibitor activity [GO:0042030] (molecular function) Sources: GOC:jl Also known as: adenosinetriphosphatase inhibitor Subtypes: DNA topoisomerase type II (double strand cut, ATP-hydrolyzing) inhibitor activity [GO:0008657], RNA helicase inhibitor activity [GO:1990119] Definition: Binds to and stops, prevents or reduces an ATP hydrolysis activity. Relationships: is a type of ATPase regulator activity [GO:0060590]; is a type of molecular function inhibitor activity [GO:0140678]; negatively regulates GO:0140657